{
  "gene_symbol": "YIPF3",
  "gene": "UniProtKB:Q9GZM5",
  "gene_name": "Protein YIPF3",
  "term_label": "Unknown molecular function",
  "term_id": "UNKNOWN:0001"
}